{
  "gene_name": "Adenosine 5'-monophosphoramidase HINT3",
  "term_label": "Unknown cellular component",
  "term_id": "UNKNOWN:0003",
  "gene": "UniProtKB:Q9NQE9",
  "gene_symbol": "HINT3"
}